mitochondrial electron transfer flavoprotein complex [GO:0017133] (cellular component) Sources: GOC:mtg_sensu, ISBN:0198506732 Relationships: is a type of electron transfer flavoprotein complex [GO:0045251]; is_a mitochondrial protein-containing complex [GO:0098798]; is part of mitochondrial matrix [GO:0005759] Definition: A protein complex located in the mitochondrion. It contains flavin adenine dinucleotide (FAD) that, together with an acyl-CoA dehydrogenase, forms a system that oxidizes an acyl-CoA molecule and reduces ubiquinone and other acceptors in the mitochondrial electron transport system.